positive regulation of activated CD4-positive, alpha-beta T cell apoptotic process [GO:1905401] (BP) Also known as: positive regulation of activated CD4-positive, alpha-beta T lymphocyte apoptotic process, positive regulation of activated CD4-positive, alpha-beta T-cell apoptotic process, positive regulation of activated CD4-positive, alpha-beta T-lymphocyte apoptotic process, up regulation of activated CD4-positive, alpha-beta T cell apoptotic process, up regulation of activated CD4-positive, alpha-beta T lymphocyte apoptotic process, up regulation of activated CD4-positive, alpha-beta T-cell apoptotic process, up regulation of activated CD4-positive, alpha-beta T-lymphocyte apoptotic process, up-regulation of activated CD4-positive, alpha-beta T cell apoptotic process, up-regulation of activated CD4-positive, alpha-beta T lymphocyte apoptotic process, up-regulation of activated CD4-positive, alpha-beta T-cell apoptotic process, up-regulation of activated CD4-positive, alpha-beta T-lymphocyte apoptotic process, upregulation of activated CD4-positive, alpha-beta T cell apoptotic process, upregulation of activated CD4-positive, alpha-beta T lymphocyte apoptotic process, upregulation of activated CD4-positive, alpha-beta T-cell apoptotic process, upregulation of activated CD4-positive, alpha-beta T-lymphocyte apoptotic process, activation of activated CD4-positive, alpha-beta T cell apoptosis, activation of activated CD4-positive, alpha-beta T cell apoptotic process, activation of activated CD4-positive, alpha-beta T lymphocyte apoptosis, activation of activated CD4-positive, alpha-beta T lymphocyte apoptotic process, activation of activated CD4-positive, alpha-beta T-cell apoptosis, activation of activated CD4-positive, alpha-beta T-cell apoptotic process, activation of activated CD4-positive, alpha-beta T-lymphocyte apoptosis, activation of activated CD4-positive, alpha-beta T-lymphocyte apoptotic process, positive regulation of activated CD4-positive, alpha-beta T cell apoptosis, positive regulation of activated CD4-positive, alpha-beta T lymphocyte apoptosis, positive regulation of activated CD4-positive, alpha-beta T-cell apoptosis, positive regulation of activated CD4-positive, alpha-beta T-lymphocyte apoptosis, up regulation of activated CD4-positive, alpha-beta T cell apoptosis, up regulation of activated CD4-positive, alpha-beta T lymphocyte apoptosis, up regulation of activated CD4-positive, alpha-beta T-cell apoptosis, up regulation of activated CD4-positive, alpha-beta T-lymphocyte apoptosis, up-regulation of activated CD4-positive, alpha-beta T cell apoptosis, up-regulation of activated CD4-positive, alpha-beta T lymphocyte apoptosis, up-regulation of activated CD4-positive, alpha-beta T-cell apoptosis, up-regulation of activated CD4-positive, alpha-beta T-lymphocyte apoptosis, upregulation of activated CD4-positive, alpha-beta T cell apoptosis, upregulation of activated CD4-positive, alpha-beta T lymphocyte apoptosis, upregulation of activated CD4-positive, alpha-beta T-cell apoptosis, upregulation of activated CD4-positive, alpha-beta T-lymphocyte apoptosis References: PMID:24187568 Sources: GOC:TermGenie, GO_REF:0000058 Relationships: is a type of positive regulation of T cell apoptotic process [GO:0070234]; is a type of regulation of activated CD4-positive, alpha-beta T cell apoptotic process [GO:1905399]; positively regulates activated CD4-positive, alpha-beta T cell apoptotic process [GO:1905398] Definition: Any process that activates or increases the frequency, rate or extent of activated CD4-positive, alpha-beta T cell apoptotic process.